{
  "gene": "UniProtKB:P20930",
  "gene_name": "Filaggrin",
  "term_label": "keratohyalin granule",
  "gene_symbol": "FLG",
  "term_id": "GO:0036457"
}